{
  "term_label": "plasma membrane",
  "gene_name": "Cdc42 effector protein 4",
  "gene": "UniProtKB:Q9H3Q1",
  "term_id": "GO:0005886",
  "gene_symbol": "CDC42EP4"
}